positive regulation of D-glucose transmembrane transport [GO:0010828] (biological process) Relationships: is a type of regulation of D-glucose transmembrane transport [GO:0010827]; is a type of positive regulation of transmembrane transport [GO:0034764]; positively regulates GO:1904659 Also known as: positive regulation of glucose transmembrane transport, positive regulation of glucose transport Sources: GOC:BHF, GOC:dph, GOC:tb Definition: Any process that increases the frequency, rate or extent of glucose transport across a membrane. Glucose transport is the directed movement of the hexose monosaccharide glucose into, out of or within a cell, or between cells, by means of some agent such as a transporter or pore. Subtypes: positive regulation of D-glucose import [GO:0046326]